type 1 cysteinyl leukotriene receptor binding [GO:0031746] (molecular function) Relationships: is a type of cysteinyl leukotriene receptor binding [GO:0031745] Also known as: type 1 cysteinyl leukotriene receptor ligand Definition: Binding to a type 1 cysteinyl leukotriene receptor. Sources: GOC:mah, GOC:nln